{
  "gene_symbol": "ESS2",
  "term_label": "Unknown biological process",
  "gene": "UniProtKB:Q96DF8",
  "term_id": "UNKNOWN:0002",
  "gene_name": "Splicing factor ESS-2 homolog"
}